{
  "term_id": "GO:0061844",
  "term_label": "antimicrobial humoral immune response mediated by antimicrobial peptide",
  "gene_symbol": "DEFB127",
  "gene": "UniProtKB:Q9H1M4",
  "gene_name": "Beta-defensin 127"
}